{
  "term_label": "cytoplasm",
  "gene_name": "AN1-type zinc finger protein 2B",
  "gene_symbol": "ZFAND2B",
  "gene": "UniProtKB:Q8WV99",
  "term_id": "GO:0005737"
}